{
  "gene_symbol": "CCR10",
  "gene": "UniProtKB:P46092",
  "term_id": "GO:0016493",
  "gene_name": "C-C chemokine receptor type 10",
  "term_label": "C-C chemokine receptor activity"
}